high-density lipoprotein particle receptor binding [GO:0070653] (molecular function) Relationships: is a type of GO:0070325 Also known as: HDL receptor binding, high-density lipoprotein receptor binding Sources: GOC:BHF, GOC:mah Definition: Binding to a high-density lipoprotein receptor.